{
  "gene_symbol": "TEX2",
  "term_id": "GO:0005783",
  "gene": "UniProtKB:Q8IWB9",
  "term_label": "endoplasmic reticulum",
  "gene_name": "Testis-expressed protein 2"
}